{
  "gene_name": "Adrenodoxin, mitochondrial",
  "gene_symbol": "FDX1",
  "gene": "UniProtKB:P10109",
  "term_label": "mitochondrion",
  "term_id": "GO:0005739"
}